{
  "term_label": "Unknown cellular component",
  "gene": "UniProtKB:Q6P531",
  "gene_symbol": "GGT6",
  "gene_name": "Glutathione hydrolase 6",
  "term_id": "UNKNOWN:0003"
}